{
  "gene": "UniProtKB:Q96F10",
  "term_id": "GO:0008080",
  "term_label": "N-acetyltransferase activity",
  "gene_name": "Thialysine N-epsilon-acetyltransferase",
  "gene_symbol": "SAT2"
}